negative regulation of cellular pH reduction [GO:0032848] (biological process) Relationships: is a type of regulation of cellular pH reduction [GO:0032847]; is a type of negative regulation of biological process [GO:0048519]; negatively regulates intracellular pH reduction [GO:0051452] Definition: Any process that stops, prevents, or reduces the frequency, rate, or extent of a process that reduces the internal pH of a cell. Sources: GOC:mah Subtypes: GO:1905527 Also known as: down regulation of cellular pH reduction, down-regulation of cellular pH reduction, downregulation of cellular pH reduction, negative regulation of cell pH reduction, negative regulation of cellular acidification, negative regulation of intracellular pH reduction, negative regulation of reduction of cellular pH, negative regulation of reduction of pH in cell, inhibition of cellular pH reduction, negative regulation of intracellular acidification